{
  "gene_symbol": "TMEM184B",
  "term_label": "membrane",
  "term_id": "GO:0016020",
  "gene_name": "Transmembrane protein 184B",
  "gene": "UniProtKB:Q9Y519"
}